{
  "gene_symbol": "ASCC3",
  "gene_name": "Activating signal cointegrator 1 complex subunit 3",
  "term_label": "3'-5' DNA helicase activity",
  "gene": "UniProtKB:Q8N3C0",
  "term_id": "GO:0043138"
}